positive regulation of heptadecane biosynthetic process [GO:1900898] (biological process) Also known as: up regulation of heptadecane biosynthetic process, up-regulation of heptadecane biosynthetic process, upregulation of heptadecane biosynthetic process, activation of heptadecane anabolism, activation of heptadecane biosynthesis, activation of heptadecane biosynthetic process, activation of heptadecane formation, activation of heptadecane synthesis, positive regulation of heptadecane anabolism, positive regulation of heptadecane biosynthesis, positive regulation of heptadecane formation, positive regulation of heptadecane synthesis, up regulation of heptadecane anabolism, up regulation of heptadecane biosynthesis, up regulation of heptadecane formation, up regulation of heptadecane synthesis, up-regulation of heptadecane anabolism, up-regulation of heptadecane biosynthesis, up-regulation of heptadecane formation, up-regulation of heptadecane synthesis, upregulation of heptadecane anabolism, upregulation of heptadecane biosynthesis, upregulation of heptadecane formation, upregulation of heptadecane synthesis Sources: GOC:TermGenie, GOC:mengo_curators Definition: Any process that activates or increases the frequency, rate or extent of heptadecane biosynthetic process. Relationships: is a type of regulation of heptadecane biosynthetic process [GO:1900896]; is a type of positive regulation of alkane biosynthetic process [GO:1901579]; positively regulates GO:1900636